negative regulation of intestinal phytosterol absorption [GO:0010949] (biological process) Definition: Any process that stops, prevents, or reduces the frequency, rate or extent of the directed movement of phytosterols into the blood by absorption from the small intestine. Sources: GOC:BHF, GOC:dph, GOC:tb Relationships: is a type of negative regulation of intestinal lipid absorption [GO:1904730]; negatively regulates intestinal phytosterol absorption [GO:0060752]